{
  "term_label": "carbonate dehydratase activity",
  "gene": "UniProtKB:Q9Y2D0",
  "term_id": "GO:0004089",
  "gene_name": "Carbonic anhydrase 5B, mitochondrial",
  "gene_symbol": "CA5B"
}